presynaptic process involved in chemical synaptic transmission [GO:0099531] (biological process) Relationships: is a type of nervous system process [GO:0050877]; is part of chemical synaptic transmission [GO:0007268]; occurs in GO:0098793 Definition: The pathway leading to secretion of a neurotransmitter from the presynapse as part of synaptic transmission. Sources: GOC:dos